regulation of extrinsic apoptotic signaling pathway via death domain receptors [GO:1902041] (biological process) References: PMID:17245429 Sources: GOC:TermGenie Also known as: regulation of death receptor-mediated apoptosis Definition: Any process that modulates the frequency, rate or extent of extrinsic apoptotic signaling pathway via death domain receptors. Relationships: is_a regulation of extrinsic apoptotic signaling pathway [GO:2001236]; regulates extrinsic apoptotic signaling pathway via death domain receptors [GO:0008625] Subtypes: negative regulation of extrinsic apoptotic signaling pathway via death domain receptors [GO:1902042], positive regulation of extrinsic apoptotic signaling pathway via death domain receptors [GO:1902043], regulation of TRAIL-activated apoptotic signaling pathway [GO:1903121]